{
  "term_id": "GO:0043235",
  "gene_name": "Platelet-derived growth factor receptor alpha",
  "gene_symbol": "PDGFRA",
  "term_label": "receptor complex",
  "gene": "UniProtKB:P16234"
}